{
  "gene_name": "Mitochondrial intermediate peptidase",
  "gene": "UniProtKB:Q99797",
  "term_id": "GO:0005739",
  "gene_symbol": "MIPEP",
  "term_label": "mitochondrion"
}